{
  "gene_symbol": "SYCE1",
  "term_id": "GO:0000795",
  "gene": "UniProtKB:Q8N0S2",
  "gene_name": "Synaptonemal complex central element protein 1",
  "term_label": "synaptonemal complex"
}